{
  "term_label": "innate immune response in mucosa",
  "gene_symbol": "H2BC5",
  "gene": "UniProtKB:P58876",
  "term_id": "GO:0002227",
  "gene_name": "Histone H2B type 1-D"
}